{
  "gene_name": "Amiloride-sensitive sodium channel subunit beta",
  "gene": "UniProtKB:P51168",
  "term_id": "GO:0015280",
  "term_label": "ligand-gated sodium channel activity",
  "gene_symbol": "SCNN1B"
}